adult fat body development [GO:0007505] (biological process) Relationships: is a type of fat body development [GO:0007503] Definition: The process whose specific outcome is the progression of the adult fat body over time, from its formation to the mature structure. Larval fat body cells that remain at eclosion degenerate in the first 2 to 4 days of adult life, leaving behind the smaller cells of the adult fat body. Sources: GOC:bf, ISBN:0879694238